{
  "term_label": "gamma-aminobutyric acid receptor clustering",
  "gene_symbol": "SHISA7",
  "gene_name": "Protein shisa-7",
  "gene": "UniProtKB:A6NL88",
  "term_id": "GO:0097112"
}